{
  "gene_name": "WASH complex subunit 1",
  "gene_symbol": "WASHC1",
  "gene": "UniProtKB:A8K0Z3",
  "term_id": "GO:0006887",
  "term_label": "exocytosis"
}